{
  "gene_symbol": "CDKN2A-DT",
  "gene_name": "Putative protein CDKN2A-DT",
  "term_id": "UNKNOWN:0003",
  "term_label": "Unknown cellular component",
  "gene": "UniProtKB:Q9UH64"
}